mannose-6-phosphate 6-reductase activity [GO:0050088] (molecular function) Relationships: is a type of GO:0016616 Definition: Catalysis of the reaction: D-mannitol 1-phosphate + NADP+ = D-mannose 6-phosphate + 3 H+ + NADPH. Also known as: 6-phosphomannose reductase activity, D-mannitol-1-phosphate:NADP+ 6-oxidoreductase activity, NADP-dependent mannose-6-P:mannitol-1-P oxidoreductase activity, NADPH-dependent M6P reductase activity, NADPH-dependent mannose 6-phosphate reductase activity, NADPH-mannose-6-P reductase activity, mannose-6-phosphate reductase activity Sources: EC:1.1.1.224, RHEA:14925